{
  "term_id": "UNKNOWN:0002",
  "gene_name": "Putative ankyrin repeat domain-containing protein 20A4",
  "gene_symbol": "ANKRD20A4P",
  "term_label": "Unknown biological process",
  "gene": "UniProtKB:Q4UJ75"
}